{
  "gene_name": "Major prion protein",
  "gene": "UniProtKB:P04156",
  "term_id": "GO:0140693",
  "term_label": "molecular condensate scaffold activity",
  "gene_symbol": "PRNP"
}